{
  "term_label": "plasma membrane",
  "gene": "UniProtKB:Q9Y6C5",
  "gene_symbol": "PTCH2",
  "gene_name": "Protein patched homolog 2",
  "term_id": "GO:0005886"
}